{
  "gene_name": "Vacuolar protein sorting-associated protein 4A",
  "gene": "UniProtKB:Q9UN37",
  "gene_symbol": "VPS4A",
  "term_label": "vacuole organization",
  "term_id": "GO:0007033"
}